{
  "term_id": "GO:0001228",
  "term_label": "DNA-binding transcription activator activity, RNA polymerase II-specific",
  "gene": "UniProtKB:Q14872",
  "gene_symbol": "MTF1",
  "gene_name": "Metal regulatory transcription factor 1"
}